negative regulation of potassium ion transmembrane transporter activity [GO:1901017] (biological process) Subtypes: negative regulation of large conductance calcium-activated potassium channel activity [GO:1902607], negative regulation of P-type sodium:potassium-exchanging transporter activity [GO:1903407], negative regulation of voltage-gated potassium channel activity [GO:1903817] Sources: GOC:BHF, GOC:TermGenie Definition: Any process that stops, prevents or reduces the frequency, rate or extent of potassium ion transmembrane transporter activity. Also known as: down regulation of potassium ion transmembrane transporter activity, down regulation of potassium transporter activity, down-regulation of potassium ion transmembrane transporter activity, down-regulation of potassium transporter activity, downregulation of potassium ion transmembrane transporter activity, downregulation of potassium transporter activity, inhibition of potassium transporter activity, negative regulation of potassium transporter activity, inhibition of potassium ion transmembrane transporter activity Relationships: is a type of negative regulation of ion transmembrane transporter activity [GO:0032413]; is a type of negative regulation of potassium ion transmembrane transport [GO:1901380]; negatively regulates potassium ion transmembrane transporter activity [GO:0015079]